mRNA splicing, via spliceosome [GO:0000398] (biological process) Also known as: mRNA splicing, pre-mRNA splicing, nuclear mRNA splicing, via spliceosome, nuclear mRNA splicing via U12-type spliceosome, nuclear mRNA splicing via U2-type spliceosome, splicing AT-AC intron, splicing GT-AG intron Sources: GOC:krc, ISBN:0198506732, ISBN:0879695897 Relationships: is_a RNA splicing, via transesterification reactions with bulged adenosine as nucleophile [GO:0000377]; is a type of GO:0006397 Subtypes: mRNA trans splicing, via spliceosome [GO:0000365], alternative mRNA splicing, via spliceosome [GO:0000380], mRNA cis splicing, via spliceosome [GO:0045292], GO:0160091 Note: Note that although the many U12-type introns have the sequence AT-AC at the intron termini, some introns with these terminal sequences are spliced by the U2-type spliceosome. The distinguishing characteristics are sequences near the 5' splice site and the branch point sequences of the intron. Note that although the majority of U2-type introns have the sequence GU-AG at the intron termini, some introns with these terminal sequences are spliced by the U12-type spliceosome. The distinguishing characteristics are sequences near the 5' splice site and the branch point sequences of the intron. Regulation: regulated by GO:0048024; negatively regulated by negative regulation of mRNA splicing, via spliceosome [GO:0048025]; RO_0002213 by positive regulation of mRNA splicing, via spliceosome [GO:0048026] Definition: The joining together of exons from one or more primary transcripts of messenger RNA (mRNA) and the excision of intron sequences, via a spliceosomal mechanism, so that mRNA consisting only of the joined exons is produced.